{
  "gene": "UniProtKB:O76062",
  "term_label": "Delta14-sterol reductase activity",
  "gene_name": "Delta(14)-sterol reductase TM7SF2",
  "term_id": "GO:0050613",
  "gene_symbol": "TM7SF2"
}